{
  "term_id": "UNKNOWN:0003",
  "term_label": "Unknown cellular component",
  "gene": "UniProtKB:Q9UDY8",
  "gene_symbol": "MALT1",
  "gene_name": "Mucosa-associated lymphoid tissue lymphoma translocation protein 1"
}